{
  "gene_name": "Nitric oxide synthase, inducible",
  "term_id": "GO:0005829",
  "gene": "UniProtKB:P35228",
  "term_label": "cytosol",
  "gene_symbol": "NOS2"
}